{
  "term_id": "GO:0009411",
  "term_label": "response to UV",
  "gene_symbol": "DDB2",
  "gene": "UniProtKB:Q92466",
  "gene_name": "DNA damage-binding protein 2"
}